cellular response to indole-3-methanol [GO:0071681] (biological process) Relationships: is a type of response to indole-3-methanol [GO:0071680]; is a type of cellular response to alcohol [GO:0097306]; is a type of GO:1901699 Definition: Any process that results in a change in state or activity of a cell (in terms of movement, secretion, enzyme production, gene expression, etc.) as a result of an indole-3-methanol stimulus. Also known as: cellular response to indole-3-carbinol Sources: GOC:mah, GOC:yaf